{
  "term_label": "positive regulation of termination of RNA polymerase II transcription, poly(A)-coupled",
  "gene": "UniProtKB:P79522",
  "gene_name": "Proline-rich protein 3",
  "gene_symbol": "PRR3",
  "term_id": "GO:2000806"
}